{
  "gene_symbol": "SERPINA9",
  "gene": "UniProtKB:Q86WD7",
  "term_label": "Unknown biological process",
  "term_id": "UNKNOWN:0002",
  "gene_name": "Serpin A9"
}